{
  "gene_name": "Sialate:O-sulfotransferase 2",
  "gene_symbol": "WSCD2",
  "term_label": "Unknown cellular component",
  "gene": "UniProtKB:Q2TBF2",
  "term_id": "UNKNOWN:0003"
}